manchette disassembly [GO:1905199] (biological process) Definition: The disaggregation of a manchette into its constituent components. References: PMID:22319670, PMID:24440897, PMID:26792866 Sources: GOC:TermGenie, GOC:krc, GO_REF:0000079 Relationships: is a type of cellular component disassembly [GO:0022411]; is part of spermatid development [GO:0007286]